negative regulation of removal of superoxide radicals [GO:1904832] (biological process) References: PMID:22836756 Sources: GOC:BHF, GOC:BHF_miRNA, GOC:TermGenie, GOC:rph, GO_REF:0000058 Also known as: down regulation of cellular detoxification of superoxide radicals, down regulation of removal of O2-, down regulation of removal of oxygen free radicals, down regulation of removal of superoxide radicals, down-regulation of cellular detoxification of superoxide radicals, down-regulation of removal of O2-, down-regulation of removal of oxygen free radicals, down-regulation of removal of superoxide radicals, downregulation of cellular detoxification of superoxide radicals, downregulation of removal of O2-, downregulation of removal of oxygen free radicals, downregulation of removal of superoxide radicals, negative regulation of cellular detoxification of superoxide radicals, negative regulation of removal of O2-, negative regulation of removal of oxygen free radicals, inhibition of cellular detoxification of superoxide radicals, inhibition of removal of O2-, inhibition of removal of oxygen free radicals, inhibition of removal of superoxide radicals Relationships: is a type of negative regulation of cellular response to oxidative stress [GO:1900408]; is a type of negative regulation of response to reactive oxygen species [GO:1901032]; is a type of regulation of removal of superoxide radicals [GO:2000121]; is a type of GO:2000378; negatively regulates removal of superoxide radicals [GO:0019430] Definition: Any process that stops, prevents or reduces the frequency, rate or extent of removal of superoxide radicals.